{
  "gene_name": "Immunoglobulin superfamily containing leucine-rich repeat protein 2",
  "gene": "UniProtKB:Q6UXK2",
  "term_id": "UNKNOWN:0001",
  "gene_symbol": "ISLR2",
  "term_label": "Unknown molecular function"
}